{
  "gene_name": "Protein FEV",
  "gene": "UniProtKB:Q99581",
  "gene_symbol": "FEV",
  "term_id": "GO:0006357",
  "term_label": "regulation of transcription by RNA polymerase II"
}